negative regulation of (1->3)-beta-D-glucan biosynthetic process [GO:0060636] (biological process) Definition: Any process that decreases the frequency, rate or extent of the chemical reactions and pathways resulting in the formation of (1->3)-beta-D-glucans. Sources: GOC:dph, GOC:tb Also known as: negative regulation of 1,3-beta-D-glucan biosynthetic process Relationships: is_a negative regulation of macromolecule biosynthetic process [GO:0010558]; is_a regulation of (1->3)-beta-D-glucan biosynthetic process [GO:0032953]; is_a negative regulation of carbohydrate metabolic process [GO:0045912]; negatively regulates (1->3)-beta-D-glucan biosynthetic process [GO:0006075]